{
  "term_id": "UNKNOWN:0003",
  "gene_symbol": "TRAJ37",
  "gene_name": "T cell receptor alpha joining 37 (Fragment)",
  "gene": "UniProtKB:A0A087X096",
  "term_label": "Unknown cellular component"
}